{
  "gene_symbol": "C8orf82",
  "gene_name": "UPF0598 protein C8orf82",
  "term_id": "UNKNOWN:0003",
  "gene": "UniProtKB:Q6P1X6",
  "term_label": "Unknown cellular component"
}